{
  "gene_name": "Kinesin-like protein KIF28P",
  "term_label": "vesicle transport along microtubule",
  "gene_symbol": "KIF28P",
  "gene": "UniProtKB:B7ZC32",
  "term_id": "GO:0047496"
}